positive regulation of microglial cell mediated cytotoxicity [GO:1904151] (biological process) References: PMID:19100238 Sources: GOC:BHF, GOC:TermGenie, GOC:nc, GO_REF:0000058 Relationships: is a type of positive regulation of leukocyte mediated cytotoxicity [GO:0001912]; is a type of positive regulation of myeloid leukocyte mediated immunity [GO:0002888]; is a type of GO:1904149; positively regulates GO:0090634 Definition: Any process that activates or increases the frequency, rate or extent of microglial cell mediated cytotoxicity. Also known as: up regulation of microglial cell mediated cytotoxicity, up-regulation of microglial cell mediated cytotoxicity, upregulation of microglial cell mediated cytotoxicity, activation of microglial cell mediated cytotoxicity